{
  "term_id": "GO:0001786",
  "gene_symbol": "GSDMB",
  "gene": "UniProtKB:Q8TAX9",
  "term_label": "phosphatidylserine binding",
  "gene_name": "Gasdermin-B"
}